non-myelinated axon ensheathment [GO:0032285] (biological process) Subtypes: GO:0032293, peripheral nervous system non-myelinated axon ensheathment [GO:0032294] Also known as: ensheathment of non-myelinated axons Sources: GOC:dgh Definition: The process in which a non-myelinating glial cell membrane closes around an axon. Relationships: is a type of axon ensheathment [GO:0008366]